{
  "term_id": "GO:0003713",
  "gene": "UniProtKB:Q13363",
  "gene_name": "C-terminal-binding protein 1",
  "term_label": "transcription coactivator activity",
  "gene_symbol": "CTBP1"
}